cellular response to very low light intensity stimulus [GO:0071488] (biological process) Sources: GOC:mah Relationships: is a type of GO:0055122; is a type of cellular response to light intensity [GO:0071484] Definition: Any process that results in a change in state or activity of a cell (in terms of movement, secretion, enzyme production, gene expression, etc.) as a result of a very low light intensity stimulus. A very low light intensity stimulus is defined as a level of electromagnetic radiation below 0.001 mmol/m2/sec.